{
  "gene": "UniProtKB:Q8IX94",
  "gene_symbol": "CTAGE4",
  "term_id": "GO:0035459",
  "gene_name": "cTAGE family member 4",
  "term_label": "vesicle cargo loading"
}